regulation of snoRNA metabolic process [GO:1903323] (biological process) Sources: GOC:TermGenie, GOC:vw, GO_REF:0000058 Subtypes: GO:1902796, negative regulation of snoRNA metabolic process [GO:1903324], positive regulation of snoRNA metabolic process [GO:1903325] Also known as: regulation of snoRNA metabolism Definition: Any process that modulates the frequency, rate or extent of snoRNA metabolic process. Relationships: is a type of regulation of RNA metabolic process [GO:0051252]; regulates sno(s)RNA metabolic process [GO:0016074]